regionalization [GO:0003002] (biological process) Definition: The pattern specification process that results in the subdivision of an axis or axes in space to define an area or volume in which specific patterns of cell differentiation will take place or in which cells interpret a specific environment. Sources: GOC:dph, GOC:isa_complete Relationships: is a type of pattern specification process [GO:0007389] Also known as: pattern formation Subtypes: tripartite regional subdivision [GO:0007351], GO:0007365, GO:0007371, imaginal disc pattern formation [GO:0007447], imaginal disc-derived wing vein specification [GO:0007474], GO:0009952, dorsal/ventral pattern formation [GO:0009953], proximal/distal pattern formation [GO:0009954], adaxial/abaxial pattern specification [GO:0009955], radial pattern formation [GO:0009956], xylem and phloem pattern formation [GO:0010051], specification of animal organ identity [GO:0010092], specification of animal organ position [GO:0010159], GO:0010160, stomatal complex patterning [GO:0010375], GO:0010622, spinal cord patterning [GO:0021511], GO:0021532, midbrain-hindbrain boundary initiation [GO:0021547], GO:0021796, forebrain regionalization [GO:0021871], telencephalon regionalization [GO:0021978], chorion-containing eggshell pattern formation [GO:0030381], cuticle pattern formation [GO:0035017], segmentation [GO:0035282], GO:0035309, GO:0045470, trichome patterning [GO:0048629], specification of plant organ number [GO:0048832], regionalization involved in semicircular canal formation [GO:0060877], limb epidermis stratification [GO:0060888], GO:0060897, left/right pattern formation [GO:0060972], bud field specification [GO:0061139], renal capsule specification [GO:0072130], GO:0080172, specification of plant organ identity [GO:0090701], specification of plant organ position [GO:0090706], centrolateral pattern formation [GO:0097353], GO:0150064, ground tissue pattern formation [GO:1990064]